{
  "term_id": "GO:0046599",
  "gene": "UniProtKB:Q96M02",
  "term_label": "regulation of centriole replication",
  "gene_symbol": "C10orf90",
  "gene_name": "(E2-independent) E3 ubiquitin-conjugating enzyme FATS"
}